{
  "term_id": "GO:0005634",
  "term_label": "nucleus",
  "gene": "UniProtKB:Q9NR20",
  "gene_name": "Dual specificity tyrosine-phosphorylation-regulated kinase 4",
  "gene_symbol": "DYRK4"
}